{
  "term_id": "GO:0008284",
  "gene_symbol": "IL23R",
  "gene_name": "Interleukin-23 receptor",
  "term_label": "positive regulation of cell population proliferation",
  "gene": "UniProtKB:Q5VWK5"
}